{
  "term_label": "RNA polymerase II preinitiation complex assembly",
  "term_id": "GO:0051123",
  "gene_symbol": "GTF2B",
  "gene": "UniProtKB:Q00403",
  "gene_name": "Transcription initiation factor IIB"
}